{
  "gene": "UniProtKB:P05787",
  "term_label": "sarcomere organization",
  "gene_symbol": "KRT8",
  "term_id": "GO:0045214",
  "gene_name": "Keratin, type II cytoskeletal 8"
}